{
  "term_label": "ciliary neurotrophic factor receptor binding",
  "gene_symbol": "OSMR",
  "gene_name": "Oncostatin-M-specific receptor subunit beta",
  "term_id": "GO:0005127",
  "gene": "UniProtKB:Q99650"
}